{
  "term_id": "GO:0005814",
  "term_label": "centriole",
  "gene_name": "WD repeat-containing protein 90",
  "gene_symbol": "WDR90",
  "gene": "UniProtKB:Q96KV7"
}